{
  "term_label": "intracellular calcium ion homeostasis",
  "gene_symbol": "ATP2A3",
  "gene_name": "Sarcoplasmic_endoplasmic reticulum calcium ATPase 3",
  "gene": "UniProtKB:Q93084",
  "term_id": "GO:0006874"
}